2',3'-cyclic-nucleotide 2'-phosphodiesterase activity [GO:0008663] (molecular function) Relationships: is a type of cyclic-nucleotide phosphodiesterase activity [GO:0004112] Also known as: 2',3'-cyclic nucleoside monophosphate phosphodiesterase, 2',3'-cyclic nucleotide phosphohydrolase, cyclic 2',3'-nucleotide phosphodiesterase, 2',3 '-cyclic AMP phosphodiesterase activity, 2',3'-cyclic AMP 2'-phosphohydrolase activity, 2',3'-cyclic nucleotidase activity, 2':3'-cyclic nucleotide phosphodiesterase:3'-nucleotidase activity, 2':3'-cyclic phosphodiesterase activity, cyclic 2',3'-nucleotide 2'-phosphodiesterase activity, cyclic phosphodiesterase:3'-nucleotidase activity, nucleoside-2',3'-cyclic-phosphate 3'-nucleotidohydrolase activity, ribonucleoside 2',3'-cyclic phosphate diesterase activity Sources: EC:3.1.4.16 Definition: Catalysis of the reaction: nucleoside 2',3'-cyclic phosphate + H2O = nucleoside 3'-phosphate.